{
  "gene_symbol": "SLC66A3",
  "term_id": "UNKNOWN:0003",
  "gene": "UniProtKB:Q8N755",
  "term_label": "Unknown cellular component",
  "gene_name": "Solute carrier family 66 member 3"
}